{
  "term_id": "UNKNOWN:0003",
  "gene_symbol": "CEND1",
  "term_label": "Unknown cellular component",
  "gene": "UniProtKB:Q8N111",
  "gene_name": "Cell cycle exit and neuronal differentiation protein 1"
}